chemoattractant activity involved in axon guidance [GO:1902379] (molecular function) Also known as: chemoattractant activity involved in axon pathfinding, chemoattractant activity involved in axon growth cone guidance, chemoattractant activity involved in axon chemotaxis Definition: Any chemoattractant activity that is involved in axon guidance. References: PMID:21658587 Sources: GOC:BHF, GOC:TermGenie, GOC:rl Relationships: is a type of GO:0042056; is part of chemoattraction of axon [GO:0061642]